{
  "term_label": "Unknown molecular function",
  "term_id": "UNKNOWN:0001",
  "gene_symbol": "TAS2R33",
  "gene": "UniProtKB:P0DSN6",
  "gene_name": "Putative taste receptor type 2 member 33"
}